{
  "gene_symbol": "VSX2",
  "term_id": "GO:0005634",
  "gene": "UniProtKB:P58304",
  "term_label": "nucleus",
  "gene_name": "Visual system homeobox 2"
}